butirosin catabolic process [GO:1901757] (biological process) Sources: GOC:TermGenie, GOC:yaf Relationships: is a type of glycoside catabolic process [GO:0016139]; is a type of polyol catabolic process [GO:0046174] Also known as: butirosin breakdown, butirosin catabolism, butirosin degradation Definition: The chemical reactions and pathways resulting in the breakdown of butirosin.